{
  "gene": "UniProtKB:Q92839",
  "term_id": "GO:0030213",
  "term_label": "hyaluronan biosynthetic process",
  "gene_symbol": "HAS1",
  "gene_name": "Hyaluronan synthase 1"
}